{
  "gene_name": "Leukocyte antigen CD37",
  "gene": "UniProtKB:P11049",
  "term_id": "UNKNOWN:0001",
  "gene_symbol": "CD37",
  "term_label": "Unknown molecular function"
}